{
  "gene_name": "Zinc finger and BTB domain-containing protein 5",
  "term_label": "DNA-binding transcription repressor activity, RNA polymerase II-specific",
  "gene_symbol": "ZBTB5",
  "term_id": "GO:0001227",
  "gene": "UniProtKB:O15062"
}